smooth muscle cell chemotaxis [GO:0071670] (biological process) Regulation: regulated by regulation of smooth muscle cell chemotaxis [GO:0071671]; negatively regulated by GO:0071672; positively regulated by GO:0071673 Relationships: is a type of smooth muscle cell migration [GO:0014909]; is_a cell chemotaxis [GO:0060326] Sources: GOC:mah Definition: The directed movement of a smooth muscle cell in response to an external stimulus.